{
  "gene_symbol": "CSMD2",
  "term_id": "UNKNOWN:0001",
  "gene_name": "CUB and sushi domain-containing protein 2",
  "term_label": "Unknown molecular function",
  "gene": "UniProtKB:Q7Z408"
}